cellobiose dehydrogenase (acceptor) activity [GO:0047735] (molecular function) Sources: EC:1.1.99.18, MetaCyc:CELLOBIOSE-DEHYDROGENASE-ACCEPTOR-RXN Relationships: is a type of oxidoreductase activity, acting on CH-OH group of donors [GO:0016614] Definition: Catalysis of the reaction: cellobiose + acceptor = cellobiono-1,5-lactone + reduced acceptor. Also known as: cellobiose dehydrogenase (quinone) activity, cellobiose-quinone oxidoreductase activity, CBOR activity, CDH activity, cellobiose dehydrogenase activity, cellobiose oxidase activity, cellobiose oxidoreductase activity, cellobiose:(acceptor) 1-oxidoreductase activity, cellobiose:acceptor 1-oxidoreductase activity, cellobiose:oxygen 1-oxidoreductase activity, phanerochaete chrysosporium cellobiose oxidoreductase activity